pre-primosome complex [GO:1990099] (cellular component) Relationships: is a type of primosome complex [GO:1990077] Definition: Any of the protein-DNA complexes that contain a DNA helicase and associated protein(s) at the origin of replication, and build up to assembling the core primosome. The associated protein(s) chaperone the helicase to the DNA, and assembly of the pre-primosome is essential for the initiation or restart of replication. Pre-primosome complexes lack a primase component. References: PMID:18179598, PMID:20129058, PMID:8663105 Sources: GOC:bhm Subtypes: GO:1990157, DnaB-DnaC-DnaT-PriA-PriB complex [GO:1990158], DnaB-DnaC-DnaT-PriA-PriC complex [GO:1990159], DnaB-DnaC-Rep-PriC complex [GO:1990160] Also known as: pre-priming complex, pre-primosome, preprimosome, preprimosome complex, prereplication complex, pre-replication complex